{
  "term_id": "UNKNOWN:0003",
  "gene_name": "Zinc finger protein 626",
  "gene_symbol": "ZNF626",
  "term_label": "Unknown cellular component",
  "gene": "UniProtKB:Q68DY1"
}